{
  "term_label": "Unknown biological process",
  "gene_name": "R3H and coiled-coil domain-containing protein 1",
  "gene": "UniProtKB:Q9Y3T6",
  "term_id": "UNKNOWN:0002",
  "gene_symbol": "R3HCC1"
}